{
  "gene_name": "Annexin A8-like protein 1",
  "term_id": "GO:0005737",
  "gene_symbol": "ANXA8L1",
  "term_label": "cytoplasm",
  "gene": "UniProtKB:Q5VT79"
}